{
  "gene": "UniProtKB:Q58FF8",
  "gene_name": "Putative heat shock protein HSP 90-beta 2",
  "term_label": "protein folding",
  "term_id": "GO:0006457",
  "gene_symbol": "HSP90AB2P"
}